{
  "term_id": "GO:0005829",
  "gene": "UniProtKB:Q05469",
  "gene_symbol": "LIPE",
  "term_label": "cytosol",
  "gene_name": "Hormone-sensitive lipase"
}